{
  "term_id": "GO:0005112",
  "gene_name": "Sushi, nidogen and EGF-like domain-containing protein 1",
  "gene_symbol": "SNED1",
  "gene": "UniProtKB:Q8TER0",
  "term_label": "Notch binding"
}